{
  "term_label": "catenin complex",
  "gene_name": "Cadherin-10",
  "gene": "UniProtKB:Q9Y6N8",
  "term_id": "GO:0016342",
  "gene_symbol": "CDH10"
}